{
  "gene": "UniProtKB:A2RUQ5",
  "gene_symbol": "TMEM132E-DT",
  "gene_name": "Uncharacterized protein TMEM132E-DT",
  "term_label": "Unknown cellular component",
  "term_id": "UNKNOWN:0003"
}